{
  "gene": "UniProtKB:O75487",
  "gene_symbol": "GPC4",
  "term_id": "GO:0099560",
  "gene_name": "Glypican-4",
  "term_label": "synaptic membrane adhesion"
}